{
  "gene_name": "Guanine nucleotide exchange factor MSS4",
  "gene": "UniProtKB:P47224",
  "gene_symbol": "RABIF",
  "term_id": "GO:0008270",
  "term_label": "zinc ion binding"
}